{
  "gene_symbol": "TCF24",
  "gene": "UniProtKB:Q7RTU0",
  "gene_name": "Transcription factor 24",
  "term_id": "GO:0006357",
  "term_label": "regulation of transcription by RNA polymerase II"
}